{
  "gene_name": "Probable C-mannosyltransferase DPY19L4",
  "term_id": "GO:0005789",
  "gene": "UniProtKB:Q7Z388",
  "gene_symbol": "DPY19L4",
  "term_label": "endoplasmic reticulum membrane"
}